{
  "term_id": "GO:0033819",
  "term_label": "lipoyl(octanoyl) transferase activity",
  "gene_symbol": "LIPT2",
  "gene_name": "Putative lipoyltransferase 2, mitochondrial",
  "gene": "UniProtKB:A6NK58"
}